negative regulation of floral organ abscission [GO:0060862] (biological process) Relationships: is a type of negative regulation of developmental process [GO:0051093]; is a type of regulation of floral organ abscission [GO:0060860]; is a type of GO:2000242; negatively regulates GO:0010227 Definition: Any process that decreases the rate, frequency, or extent of floral organ abscission, the controlled shedding of floral organs. Sources: GOC:dph, GOC:sdb_2009, GOC:tb